vitamin K biosynthetic process [GO:0042371] (biological process) Definition: The chemical reactions and pathways resulting in the formation of any of the forms of vitamin K, quinone-derived vitamins which are involved in the synthesis of blood-clotting factors in mammals. References: PMID:24489112 Sources: GOC:jl, https://en.wikipedia.org/wiki/Vitamin_K Also known as: naphthoquinone metabolic process, naphthoquinone metabolism, vitamin K anabolism, vitamin K biosynthesis, vitamin K formation, vitamin K synthesis Relationships: is a type of ketone biosynthetic process [GO:0042181]; is a type of fat-soluble vitamin biosynthetic process [GO:0042362]; is a type of GO:0042373 Subtypes: phylloquinone biosynthetic process [GO:0042372]